medium-chain fatty acid metabolic process [GO:0051791] (biological process) Definition: The chemical reactions and pathways involving a medium-chain fatty acid. A medium-chain fatty acid has an aliphatic tail containing 6 to 12 carbons. Also known as: medium chain fatty acid metabolic process, medium chain fatty acid metabolism, medium-chain fatty acid metabolism Sources: Wikipedia:Fatty_acid_metabolisms Subtypes: GO:0048252, GO:0051792, GO:0051793 Note: While there is not universal consensus on the lengths of short-, medium-, long- and very-long-chain fatty acids, the GO uses the definitions in ChEBI (see CHEBI:26666, CHEBI:59554, CHEBI:15904 and CHEBI:27283). Relationships: is a type of fatty acid metabolic process [GO:0006631]